{
  "gene": "UniProtKB:Q9H1B5",
  "term_label": "heparan sulfate proteoglycan biosynthetic process",
  "gene_symbol": "XYLT2",
  "gene_name": "Xylosyltransferase 2",
  "term_id": "GO:0015012"
}